{
  "gene": "UniProtKB:Q9H7E2",
  "term_id": "GO:0005634",
  "term_label": "nucleus",
  "gene_symbol": "TDRD3",
  "gene_name": "Tudor domain-containing protein 3"
}